{
  "gene": "UniProtKB:Q8NGP6",
  "term_label": "sensory perception of smell",
  "gene_name": "Olfactory receptor 5M8",
  "gene_symbol": "OR5M8",
  "term_id": "GO:0007608"
}